{
  "gene": "UniProtKB:Q96LR5",
  "term_id": "GO:0070979",
  "gene_symbol": "UBE2E2",
  "term_label": "protein K11-linked ubiquitination",
  "gene_name": "Ubiquitin-conjugating enzyme E2 E2"
}